{
  "gene": "UniProtKB:Q86XF0",
  "gene_symbol": "DHFR2",
  "term_id": "GO:0046655",
  "gene_name": "Dihydrofolate reductase 2, mitochondrial",
  "term_label": "folic acid metabolic process"
}